{
  "gene_symbol": "OPN1LW",
  "term_label": "photoreceptor outer segment",
  "gene_name": "Long-wave-sensitive opsin 1",
  "term_id": "GO:0001750",
  "gene": "UniProtKB:P04000"
}